{
  "term_id": "UNKNOWN:0001",
  "gene_symbol": "FBXO15",
  "gene": "UniProtKB:Q8NCQ5",
  "gene_name": "F-box only protein 15",
  "term_label": "Unknown molecular function"
}